tRNA import into mitochondrion [GO:0016031] (biological process) Definition: The process in which a tRNA is transported from the cytosol into the mitochondrial matrix. Also known as: cytoplasmic tRNA import into mitochondria, cytoplasmic tRNA transport into mitochondrion, cytoplasmic tRNA, mitochondrial import, cytoplasmic tRNA import into mitochondrion, mitochondrial import of cytoplasmic tRNA, nuclear-encoded tRNA import into mitochondrion Relationships: is a type of RNA import into mitochondrion [GO:0035927]; is a type of tRNA transport [GO:0051031] References: PMID:10988073, PMID:11121736 Sources: GOC:ma